{
  "term_id": "GO:0005634",
  "term_label": "nucleus",
  "gene": "UniProtKB:P05114",
  "gene_symbol": "HMGN1",
  "gene_name": "Non-histone chromosomal protein HMG-14"
}